{
  "gene_name": "T cell receptor alpha joining 6 (Fragment)",
  "term_label": "Unknown biological process",
  "term_id": "UNKNOWN:0002",
  "gene": "UniProtKB:A0A075B6Z3",
  "gene_symbol": "TRAJ6"
}